{
  "gene_symbol": "HERC5",
  "gene": "UniProtKB:Q9UII4",
  "term_id": "GO:0042296",
  "term_label": "ISG15 transferase activity",
  "gene_name": "E3 ISG15--protein ligase HERC5"
}